{
  "term_id": "GO:0010879",
  "gene_name": "StAR-related lipid transfer protein 4",
  "gene": "UniProtKB:Q96DR4",
  "term_label": "cholesterol transport involved in cholesterol storage",
  "gene_symbol": "STARD4"
}